{
  "gene": "UniProtKB:P48549",
  "gene_symbol": "KCNJ3",
  "term_id": "GO:0005886",
  "gene_name": "G protein-activated inward rectifier potassium channel 1",
  "term_label": "plasma membrane"
}